{
  "gene_symbol": "TNFRSF4",
  "term_id": "GO:0009897",
  "gene_name": "Tumor necrosis factor receptor superfamily member 4",
  "gene": "UniProtKB:P43489",
  "term_label": "external side of plasma membrane"
}